{
  "gene": "UniProtKB:Q8IZS6",
  "term_label": "cytoplasmic dynein complex",
  "gene_symbol": "DYNLT2",
  "term_id": "GO:0005868",
  "gene_name": "Dynein light chain Tctex-type protein 2"
}